{
  "gene_symbol": "TRERF1",
  "term_label": "histone deacetylase complex",
  "gene": "UniProtKB:Q96PN7",
  "gene_name": "Transcriptional-regulating factor 1",
  "term_id": "GO:0000118"
}